{
  "term_id": "GO:0035758",
  "gene_symbol": "CCR7",
  "term_label": "chemokine (C-C motif) ligand 21 binding",
  "gene_name": "C-C chemokine receptor type 7",
  "gene": "UniProtKB:P32248"
}